{
  "gene": "UniProtKB:Q9BYZ6",
  "term_id": "GO:0005856",
  "gene_name": "Rho-related BTB domain-containing protein 2",
  "term_label": "cytoskeleton",
  "gene_symbol": "RHOBTB2"
}